glutathione transferase activity [GO:0004364] (molecular function) Also known as: glutathione conjugation reaction, RX:glutathione R-transferase activity, S-(hydroxyalkyl)glutathione lyase activity, glutathione S-alkyl transferase activity, glutathione S-alkyltransferase activity, glutathione S-aralkyltransferase activity, glutathione S-aryltransferase activity, glutathione S-transferase activity Definition: Catalysis of the reaction: R-X + glutathione = H-X + R-S-glutathione. R may be an aliphatic, aromatic or heterocyclic group; X may be a sulfate, nitrile or halide group. Sources: EC:2.5.1.18 Relationships: is a type of transferase activity, transferring alkyl or aryl (other than methyl) groups [GO:0016765]